{
  "gene_name": "Probable G-protein coupled receptor 153",
  "term_label": "Unknown biological process",
  "gene_symbol": "GPR153",
  "gene": "UniProtKB:Q6NV75",
  "term_id": "UNKNOWN:0002"
}